phosphatidic acid binding [GO:0070300] (molecular function) Also known as: phosphatidate binding Definition: Binding to phosphatidic acid, any of a class of glycerol phosphate in which both the remaining hydroxyl groups of the glycerol moiety are esterified with fatty acids. Relationships: is a type of phospholipid binding [GO:0005543]; is a type of anion binding [GO:0043168] Sources: CHEBI:16337, GOC:jp, ISBN:0198506732